phenylcoumaran benzylic ether reductase activity [GO:0032442] (molecular function) Definition: Catalysis of the NADPH-dependent 7-O-4' reduction of phenylcoumaran lignans to the corresponding diphenols; for example, catalysis of the reaction: dehydrodiconiferyl alcohol + NADPH + H+ = isodihydrodehydrodiconiferyl alcohol + NADP+. Also known as: PCBER activity Relationships: is a type of GO:0016616 References: PMID:11030549, PMID:13129921